{
  "term_label": "cytoplasm",
  "gene_symbol": "NEDD4",
  "term_id": "GO:0005737",
  "gene": "UniProtKB:P46934",
  "gene_name": "E3 ubiquitin-protein ligase NEDD4"
}